iota-carrageenase activity [GO:0033952] (molecular function) Definition: Catalysis of the endohydrolysis of 1,4-beta-D-linkages between D-galactose 4-sulfate and 3,6-anhydro-D-galactose-2-sulfate in iota-carrageenans. Relationships: is a type of GO:0004553 Sources: EC:3.2.1.157 Also known as: iota-carrageenan 4-beta-D-glycanohydrolase (configuration-inverting) activity